uracil-5-carboxylate decarboxylase activity [GO:0050382] (molecular function) Also known as: uracil-5-carboxylate carboxy-lyase (uracil-forming), uracil-5-carboxylate carboxy-lyase activity, uracil-5-carboxylic acid decarboxylase activity Definition: Catalysis of the reaction: H+ + uracil 5-carboxylate = CO2 + uracil. Relationships: is a type of carboxy-lyase activity [GO:0016831] Sources: EC:4.1.1.66, RHEA:17685